{
  "gene_symbol": "SQSTM1",
  "gene": "UniProtKB:Q13501",
  "gene_name": "Sequestosome-1",
  "term_id": "GO:0000423",
  "term_label": "mitophagy"
}